mature B cell differentiation involved in immune response [GO:0002313] (BP) Sources: GOC:jal Subtypes: germinal center B cell differentiation [GO:0002314], marginal zone B cell differentiation [GO:0002315], follicular B cell differentiation [GO:0002316], plasma cell differentiation [GO:0002317], memory B cell differentiation [GO:0002319] Definition: The process in which a naive B cell acquires the specialized features of a mature or memory B cell during an immune response. Note: Note that immunologists typically use the word 'development' to refer to cells of B or T cell lineages undergoing the process that GO describes as 'cell differentiation'. Also known as: mature B cell development involved in immune response, mature B cell differentiation during immune response, mature B lymphocyte differentiation during immune response, mature B-cell differentiation during immune response, mature B-lymphocyte differentiation during immune response Relationships: is a type of B cell activation involved in immune response [GO:0002312]; is a type of GO:0002335